{
  "term_id": "UNKNOWN:0002",
  "term_label": "Unknown biological process",
  "gene_symbol": "SLC66A1",
  "gene": "UniProtKB:Q6ZP29",
  "gene_name": "Lysosomal amino acid transporter 1 homolog"
}